{
  "gene_symbol": "NUP133",
  "term_id": "GO:0006606",
  "term_label": "protein import into nucleus",
  "gene_name": "Nuclear pore complex protein Nup133",
  "gene": "UniProtKB:Q8WUM0"
}